ion channel regulator activity [GO:0099106] (molecular function) Subtypes: calcium channel regulator activity [GO:0005246], ion channel inhibitor activity [GO:0008200], potassium channel regulator activity [GO:0015459], sodium channel regulator activity [GO:0017080], chloride channel regulator activity [GO:0017081] Definition: Modulates the activity of a channel via direct interaction with it. A channel catalyzes energy-independent facilitated diffusion, mediated by passage of a solute through a transmembrane aqueous pore or channel. Sources: GOC:dos Relationships: is a type of channel regulator activity [GO:0016247]; regulates monoatomic ion channel activity [GO:0005216]